UDP-glucuronate 4-epimerase activity [GO:0050378] (molecular function) Also known as: UDP glucuronic epimerase activity, UDP-D-galacturonic acid 4-epimerase activity, UDP-galacturonate 4-epimerase activity, UDPglucuronate 4-epimerase activity, uridine diphospho-D-galacturonic acid, uridine diphosphoglucuronate epimerase activity, uridine diphosphoglucuronic epimerase activity Relationships: is a type of racemase and epimerase activity, acting on carbohydrates and derivatives [GO:0016857] Definition: Catalysis of the reaction: UDP-alpha-D-glucuronate = UDP-alpha-D-galacturonate. Note: Note that this term has a MetaCyc pathway reference as the pathway only has a single step. Sources: EC:5.1.3.6, RHEA:11404